{
  "gene_name": "Phospholipid-transporting ATPase IF",
  "term_id": "GO:0055037",
  "term_label": "recycling endosome",
  "gene": "UniProtKB:Q9Y2G3",
  "gene_symbol": "ATP11B"
}